{
  "gene": "UniProtKB:O14786",
  "gene_symbol": "NRP1",
  "term_id": "GO:0009611",
  "gene_name": "Neuropilin-1",
  "term_label": "response to wounding"
}